{
  "gene": "UniProtKB:P48739",
  "term_id": "GO:0008526",
  "gene_name": "Phosphatidylinositol transfer protein beta isoform",
  "term_label": "phosphatidylinositol transfer activity",
  "gene_symbol": "PITPNB"
}